{
  "gene_symbol": "CD244",
  "term_id": "GO:0009897",
  "gene_name": "Natural killer cell receptor 2B4",
  "gene": "UniProtKB:Q9BZW8",
  "term_label": "external side of plasma membrane"
}